negative regulation of interleukin-5 production [GO:0032714] (biological process) Sources: GOC:mah Also known as: down regulation of interleukin-5 production, down-regulation of interleukin-5 production, downregulation of interleukin-5 production, negative regulation of IL-5 production, inhibition of interleukin-5 production, negative regulation of interleukin-5 biosynthetic process, negative regulation of interleukin-5 secretion Definition: Any process that stops, prevents, or reduces the frequency, rate, or extent of interleukin-5 production. Relationships: is a type of negative regulation of cytokine production [GO:0001818]; is a type of GO:0032674; negatively regulates interleukin-5 production [GO:0032634]